{
  "term_id": "GO:0031012",
  "gene_name": "Heparanase",
  "term_label": "extracellular matrix",
  "gene": "UniProtKB:Q9Y251",
  "gene_symbol": "HPSE"
}